{
  "gene": "UniProtKB:Q96I27",
  "term_label": "RNA polymerase II transcription regulatory region sequence-specific DNA binding",
  "gene_name": "Zinc finger protein 625",
  "gene_symbol": "ZNF625",
  "term_id": "GO:0000977"
}